{
  "gene_name": "Protein PIGBOS1",
  "gene": "UniProtKB:A0A0B4J2F0",
  "gene_symbol": "PIGBOS1",
  "term_id": "UNKNOWN:0002",
  "term_label": "Unknown biological process"
}